{
  "term_id": "GO:0045214",
  "term_label": "sarcomere organization",
  "gene_symbol": "TNNT3",
  "gene_name": "Troponin T, fast skeletal muscle",
  "gene": "UniProtKB:P45378"
}